{
  "gene": "UniProtKB:P19429",
  "gene_name": "Troponin I, cardiac muscle",
  "term_id": "GO:0060048",
  "gene_symbol": "TNNI3",
  "term_label": "cardiac muscle contraction"
}